{
  "gene_name": "Endogenous retrovirus group K member 7 Pol protein",
  "gene_symbol": "ERVK-7",
  "term_label": "RNA stem-loop binding",
  "term_id": "GO:0035613",
  "gene": "UniProtKB:P63135"
}